tRNA (cytidine(34)-2'-O)-methyltransferase activity [GO:0141098] (molecular function) References: PMID:31943105 Sources: RHEA:43084 Definition: Catalysis of the reaction: cytidine(34) in tRNA + S-adenosyl-L-methionine = 2'-O-methylcytidine(34) in tRNA + H+ + S-adenosyl-L-homocysteine. Also known as: tRNA (cytidine 34-2'-O)-methyltransferase activity Relationships: is a type of tRNA (cytidine) methyltransferase activity [GO:0016427]